{
  "term_id": "GO:0005634",
  "gene_name": "Homeobox protein DLX-1",
  "term_label": "nucleus",
  "gene_symbol": "DLX1",
  "gene": "UniProtKB:P56177"
}